{
  "gene_name": "NADH dehydrogenase [ubiquinone] iron-sulfur protein 3, mitochondrial",
  "gene": "UniProtKB:O75489",
  "term_label": "respiratory chain complex I",
  "gene_symbol": "NDUFS3",
  "term_id": "GO:0045271"
}